{
  "term_id": "UNKNOWN:0002",
  "gene": "UniProtKB:A0A8V8TPW1",
  "gene_name": "Uncharacterized protein",
  "gene_symbol": "A0A8V8TPW1",
  "term_label": "Unknown biological process"
}